{
  "term_id": "GO:0007283",
  "gene_name": "Testis development-related protein",
  "gene": "UniProtKB:Q86YL5",
  "term_label": "spermatogenesis",
  "gene_symbol": "TDRP"
}